metanephric proximal tubule development [GO:0072237] (BP) Definition: The process whose specific outcome is the progression of the metanephric proximal tubule over time, from its formation to the mature structure. The metanephric proximal tubule is a metanephric nephron tubule that connects Bowman's capsule to the descending thin limb of the loop of Henle in the metanephros. It has a brush border epithelial morphology. Sources: GOC:mtg_kidney_jan10 Relationships: is a type of proximal tubule development [GO:0072014]; is a type of GO:0072234